{
  "gene_symbol": "GABRP",
  "gene": "UniProtKB:O00591",
  "gene_name": "Gamma-aminobutyric acid receptor subunit pi",
  "term_id": "GO:0051932",
  "term_label": "synaptic transmission, GABAergic"
}